{
  "term_label": "Unknown biological process",
  "gene_name": "Cilia- and flagella-associated protein 299",
  "gene": "UniProtKB:Q6V702",
  "gene_symbol": "CFAP299",
  "term_id": "UNKNOWN:0002"
}